{
  "gene": "UniProtKB:Q8TF09",
  "term_label": "dynein intermediate chain binding",
  "gene_name": "Dynein light chain roadblock-type 2",
  "gene_symbol": "DYNLRB2",
  "term_id": "GO:0045505"
}